cellular response to catechin [GO:1902169] (biological process) Definition: Any process that results in a change in state or activity of a cell (in terms of movement, secretion, enzyme production, gene expression, etc.) as a result of a catechin stimulus. References: PMID:23516620 Sources: GOC:TermGenie, GOC:rjd Relationships: is a type of response to catechin [GO:1902168]; is a type of cellular response to flavonoid [GO:1905396]; is a type of GO:1905546